{
  "term_id": "GO:0003779",
  "gene_symbol": "PDLIM4",
  "gene": "UniProtKB:P50479",
  "gene_name": "PDZ and LIM domain protein 4",
  "term_label": "actin binding"
}